{
  "gene": "UniProtKB:Q68EM7",
  "gene_name": "Rho GTPase-activating protein 17",
  "term_label": "GTPase activator activity",
  "term_id": "GO:0005096",
  "gene_symbol": "ARHGAP17"
}